{
  "term_label": "positive regulation of synaptic transmission, glutamatergic",
  "term_id": "GO:0051968",
  "gene": "UniProtKB:Q9UBN1",
  "gene_name": "Voltage-dependent calcium channel gamma-4 subunit",
  "gene_symbol": "CACNG4"
}